{
  "gene_symbol": "SIX3",
  "term_id": "GO:0005634",
  "gene_name": "Homeobox protein SIX3",
  "gene": "UniProtKB:O95343",
  "term_label": "nucleus"
}